{
  "term_id": "GO:0006661",
  "gene_name": "CDP-diacylglycerol--inositol 3-phosphatidyltransferase",
  "gene": "UniProtKB:O14735",
  "term_label": "phosphatidylinositol biosynthetic process",
  "gene_symbol": "CDIPT"
}